{
  "gene": "UniProtKB:Q5JXC2",
  "term_id": "UNKNOWN:0003",
  "gene_name": "Migration and invasion-inhibitory protein",
  "term_label": "Unknown cellular component",
  "gene_symbol": "MIIP"
}